{
  "gene_symbol": "TCF19",
  "gene": "UniProtKB:Q9Y242",
  "term_label": "Unknown molecular function",
  "term_id": "UNKNOWN:0001",
  "gene_name": "Transcription factor 19"
}